o-orsellinic acid biosynthetic process [GO:1900584] (biological process) Regulation: regulated by regulation of o-orsellinic acid biosynthetic process [GO:1900698]; RO_0002212 by negative regulation of o-orsellinic acid biosynthetic process [GO:1900699]; positively regulated by positive regulation of o-orsellinic acid biosynthetic process [GO:1900700] Definition: The chemical reactions and pathways resulting in the formation of o-orsellinic acid. Relationships: is a type of GO:0042537; is a type of secondary metabolite biosynthetic process [GO:0044550]; is a type of phenol-containing compound biosynthetic process [GO:0046189]; is a type of GO:0072330 Sources: GOC:TermGenie, GOC:di Also known as: o-orsellinic acid anabolism, o-orsellinic acid biosynthesis, o-orsellinic acid formation, o-orsellinic acid synthesis